{
  "gene_name": "Myb-related protein B",
  "gene_symbol": "MYBL2",
  "gene": "UniProtKB:P10244",
  "term_id": "GO:0000981",
  "term_label": "DNA-binding transcription factor activity, RNA polymerase II-specific"
}